{
  "term_label": "plasma membrane",
  "gene_symbol": "RGS3",
  "gene": "UniProtKB:P49796",
  "gene_name": "Regulator of G-protein signaling 3",
  "term_id": "GO:0005886"
}